{
  "gene_name": "Myelin proteolipid protein",
  "gene": "UniProtKB:P60201",
  "term_id": "GO:0005886",
  "term_label": "plasma membrane",
  "gene_symbol": "PLP1"
}